plant epidermis development [GO:0090558] (biological process) Subtypes: stomatal complex development [GO:0010374] Definition: The process whose specific outcome is the progression of the plant epidermis over time, from its formation to the mature structure. Relationships: is a type of tissue development [GO:0009888] Sources: GOC:tb